{
  "term_label": "cytochrome-c oxidase activity",
  "gene_symbol": "MT-CO2",
  "gene": "UniProtKB:P00403",
  "gene_name": "Cytochrome c oxidase subunit 2",
  "term_id": "GO:0004129"
}